{
  "term_id": "GO:0030992",
  "gene_symbol": "IFT56",
  "gene": "UniProtKB:A0AVF1",
  "gene_name": "Intraflagellar transport protein 56",
  "term_label": "intraciliary transport particle B"
}